regulation of antigen processing and presentation of lipid antigen via MHC class Ib [GO:0002598] (biological process) Relationships: is a type of GO:0002592; regulates antigen processing and presentation of lipid antigen via MHC class Ib [GO:0048003] Sources: GOC:add Subtypes: negative regulation of antigen processing and presentation of lipid antigen via MHC class Ib [GO:0002599], GO:0002600 Also known as: regulation of lipid antigen processing and presentation via MHC class Ib Definition: Any process that modulates the frequency, rate, or extent of antigen processing and presentation of lipid antigen via MHC class Ib.